{
  "gene_symbol": "CTSH",
  "gene_name": "Pro-cathepsin H",
  "term_label": "extracellular space",
  "term_id": "GO:0005615",
  "gene": "UniProtKB:P09668"
}